negative regulation of chemokine activity [GO:1900137] (biological process) Sources: GOC:TermGenie Relationships: is a type of negative regulation of cell migration [GO:0030336]; is a type of negative regulation of chemotaxis [GO:0050922]; is a type of negative regulation of cytokine activity [GO:0060302]; is a type of regulation of chemokine activity [GO:1900136]; negatively regulates GO:0008009 Definition: Any process that stops, prevents or reduces the frequency, rate or extent of chemokine activity. Also known as: down regulation of chemokine activity, down-regulation of chemokine activity, downregulation of chemokine activity, inhibition of chemokine activity